{
  "gene": "UniProtKB:Q5JS37",
  "gene_name": "NHL repeat-containing protein 3",
  "term_id": "GO:0061630",
  "gene_symbol": "NHLRC3",
  "term_label": "ubiquitin protein ligase activity"
}